{
  "gene": "UniProtKB:Q86TJ5",
  "gene_symbol": "ZNF554",
  "term_label": "nucleus",
  "term_id": "GO:0005634",
  "gene_name": "Zinc finger protein 554"
}